{
  "term_label": "cellular response to estradiol stimulus",
  "gene": "UniProtKB:P30874",
  "gene_name": "Somatostatin receptor type 2",
  "gene_symbol": "SSTR2",
  "term_id": "GO:0071392"
}